{
  "gene_name": "E3 ubiquitin-protein ligase RNF138",
  "gene": "UniProtKB:Q8WVD3",
  "gene_symbol": "RNF138",
  "term_label": "site of double-strand break",
  "term_id": "GO:0035861"
}